peptidyl-histidine phosphorylation [GO:0018106] (biological process) Sources: RESID:AA0035, RESID:AA0036 Definition: The phosphorylation of peptidyl-histidine to form peptidyl-1'-phospho-L-histidine (otherwise known as tau-phosphohistidine, tele-phosphohistidine) or peptidyl-3'-phospho-L-histidine (otherwise known as pi-phosphohistidine, pros-phosphohistidine). Relationships: is a type of GO:0006468; is a type of peptidyl-histidine modification [GO:0018202]